{
  "gene_name": "Putative TBC1 domain family member 29",
  "gene_symbol": "TBC1D29P",
  "term_id": "UNKNOWN:0002",
  "gene": "UniProtKB:Q9UFV1",
  "term_label": "Unknown biological process"
}